{
  "gene_name": "G patch domain-containing protein 4",
  "term_label": "nucleolus",
  "gene": "UniProtKB:Q5T3I0",
  "gene_symbol": "GPATCH4",
  "term_id": "GO:0005730"
}